{
  "term_label": "low-density lipoprotein particle receptor activity",
  "gene_symbol": "CD36",
  "term_id": "GO:0005041",
  "gene": "UniProtKB:P16671",
  "gene_name": "Platelet glycoprotein 4"
}